{
  "gene": "UniProtKB:Q8NFR7",
  "gene_symbol": "CCDC148",
  "term_id": "UNKNOWN:0002",
  "gene_name": "Coiled-coil domain-containing protein 148",
  "term_label": "Unknown biological process"
}